{
  "gene_name": "Plastin-2",
  "term_id": "GO:0005884",
  "gene_symbol": "LCP1",
  "term_label": "actin filament",
  "gene": "UniProtKB:P13796"
}